4-hydroxy-L-isoleucine dehydrogenase activity [GO:0102394] (molecular function) References: PMID:21069315 Sources: GOC:pz Relationships: is a type of oxidoreductase activity, acting on the CH-OH group of donors, NAD or NADP as acceptor [GO:0016616] Definition: Catalysis of the reaction: (2S,3R,4S)-4-hydroxy-L-isoleucine + NAD = (2S,3R)-2-amino-3-methyl-4-ketopentanoate + NADH + H+.